{
  "term_id": "GO:0021955",
  "gene_name": "Spastin",
  "gene": "UniProtKB:Q9UBP0",
  "term_label": "central nervous system neuron axonogenesis",
  "gene_symbol": "SPAST"
}